{
  "gene_name": "Formimidoyltransferase-cyclodeaminase",
  "gene": "UniProtKB:O95954",
  "term_id": "GO:0030409",
  "gene_symbol": "FTCD",
  "term_label": "glutamate formimidoyltransferase activity"
}